{
  "gene": "UniProtKB:P24386",
  "gene_name": "Rab proteins geranylgeranyltransferase component A 1",
  "term_id": "GO:0006612",
  "term_label": "protein targeting to membrane",
  "gene_symbol": "CHM"
}